{
  "gene": "UniProtKB:P36222",
  "gene_symbol": "CHI3L1",
  "term_label": "chitin catabolic process",
  "term_id": "GO:0006032",
  "gene_name": "Chitinase-3-like protein 1"
}